{
  "gene": "UniProtKB:O60258",
  "gene_name": "Fibroblast growth factor 17",
  "term_label": "fibroblast growth factor receptor signaling pathway",
  "gene_symbol": "FGF17",
  "term_id": "GO:0008543"
}